{
  "term_label": "nucleolus",
  "gene_symbol": "EIF4A3",
  "gene_name": "Eukaryotic initiation factor 4A-III",
  "gene": "UniProtKB:P38919",
  "term_id": "GO:0005730"
}